{
  "gene_name": "Phosphate-regulating neutral endopeptidase PHEX",
  "term_label": "protein processing",
  "gene_symbol": "PHEX",
  "gene": "UniProtKB:P78562",
  "term_id": "GO:0016485"
}